{
  "gene_name": "Aldehyde dehydrogenase, mitochondrial",
  "term_label": "aldehyde dehydrogenase (NAD+) activity",
  "gene": "UniProtKB:P05091",
  "gene_symbol": "ALDH2",
  "term_id": "GO:0004029"
}